ergothioneine metabolic process [GO:0052698] (biological process) Subtypes: ergothioneine biosynthetic process [GO:0052699], ergothioneine catabolic process [GO:0052700] Relationships: is a type of sulfur amino acid metabolic process [GO:0000096]; is a type of GO:0006577 Also known as: (2S)-3-(2-mercapto-1H-imidazol-5-yl)-2-(trimethylazaniumyl)propanoate metabolic process, 2-mercaptoergothioneine trimethylbetaine metabolic process, 2-mercaptoergothioneine trimethylbetaine metabolism, ergothioneine metabolism Sources: Wikipedia:Ergothioneine Definition: The chemical reactions and pathways involving ergothioneine, a naturally occurring metabolite of histidine with antioxidant properties.